establishment of secretory granule localization [GO:0032254] (biological process) Also known as: establishment of secretory granule localisation Relationships: is a type of establishment of vesicle localization [GO:0051650]; is part of secretory granule localization [GO:0032252] Sources: GOC:mah Subtypes: establishment of dense core granule localization [GO:0032256] Definition: The directed movement of a secretory granule to a specific location.